{
  "gene": "UniProtKB:A0A0B4J272",
  "gene_symbol": "TRAV24",
  "gene_name": "T cell receptor alpha variable 24",
  "term_id": "UNKNOWN:0001",
  "term_label": "Unknown molecular function"
}